{
  "term_label": "regulation of transcription by RNA polymerase II",
  "gene": "UniProtKB:P0CG40",
  "gene_symbol": "SP9",
  "term_id": "GO:0006357",
  "gene_name": "Transcription factor Sp9"
}